{
  "gene_symbol": "ATP6V1B2",
  "gene": "UniProtKB:P21281",
  "term_label": "proton transmembrane transport",
  "gene_name": "V-type proton ATPase subunit B, brain isoform",
  "term_id": "GO:1902600"
}